{
  "term_label": "plasma membrane",
  "gene": "UniProtKB:P36269",
  "gene_name": "Glutathione hydrolase 5 proenzyme",
  "term_id": "GO:0005886",
  "gene_symbol": "GGT5"
}